polyvinyl-alcohol oxidase activity [GO:0050209] (molecular function) Definition: Catalysis of the reaction: polyvinyl alcohol + O2 = oxidized polyvinyl alcohol + H2O2. Sources: EC:1.1.3.30, MetaCyc:POLYVINYL-ALCOHOL-OXIDASE-RXN Also known as: PVA oxidase activity, dehydrogenase, polyvinyl alcohol, polyvinyl-alcohol:oxygen oxidoreductase activity Relationships: is a type of oxidoreductase activity, acting on the CH-OH group of donors, oxygen as acceptor [GO:0016899]